interleukin-22 receptor binding [GO:0045518] (MF) Definition: Binding to an interleukin-22 receptor. Also known as: IL-22, interleukin-22 receptor ligand Sources: GOC:go_curators Relationships: is_a GO:0005126